{
  "gene_symbol": "TSLP",
  "gene_name": "Thymic stromal lymphopoietin",
  "gene": "UniProtKB:Q969D9",
  "term_id": "GO:0005125",
  "term_label": "cytokine activity"
}